dTDP-4-dehydrorhamnose reductase activity [GO:0008831] (molecular function) Also known as: TDP-4-keto-rhamnose reductase activity, dTDP-4-keto-L-rhamnose reductase activity, dTDP-4-ketorhamnose reductase activity, dTDP-6-deoxy-L-mannose dehydrogenase activity, dTDP-6-deoxy-L-mannose:NADP+ 4-oxidoreductase activity, reductase, thymidine diphospho-4-ketorhamnose, thymidine diphospho-4-ketorhamnose reductase activity Definition: Catalysis of the reaction: dTDP-6-deoxy-L-mannose + NADP+ = dTDP-4-dehydro-6-deoxy-L-mannose + H+ + NADPH. Relationships: is a type of oxidoreductase activity, acting on the CH-OH group of donors, NAD or NADP as acceptor [GO:0016616] Sources: EC:1.1.1.133, RHEA:21796